Cul4A-RING E3 ubiquitin ligase complex [GO:0031464] (cellular component) Definition: A ubiquitin ligase complex in which a cullin from the Cul4A subfamily and a RING domain protein form the catalytic core; substrate specificity is conferred by an adaptor protein. References: PMID:15571813, PMID:15688063 Also known as: CDL4 complex, CRL4 complex, DCX complex, cullin-RING ligase 4A, VDC complex, SCF4 complex Relationships: is a type of Cul4-RING E3 ubiquitin ligase complex [GO:0080008]